dalcochinase activity [GO:0102954] (molecular function) Relationships: is a type of GO:0004553 Definition: Catalysis of the reaction: dalcochinin-8'-O-beta-glucoside + H2O = dalcochinin + D-glucopyranose. References: PMID:16814564 Sources: GOC:pz